{
  "term_label": "plasma membrane",
  "gene_symbol": "CEACAM7",
  "gene_name": "Carcinoembryonic antigen-related cell adhesion molecule 7",
  "gene": "UniProtKB:Q14002",
  "term_id": "GO:0005886"
}